{
  "gene_name": "Keratin, type I cuticular Ha2",
  "gene": "UniProtKB:Q14532",
  "term_label": "keratin filament",
  "gene_symbol": "KRT32",
  "term_id": "GO:0045095"
}